{
  "term_id": "GO:0050830",
  "term_label": "defense response to Gram-positive bacterium",
  "gene_name": "Inactive ribonuclease-like protein 10",
  "gene_symbol": "RNASE10",
  "gene": "UniProtKB:Q5GAN6"
}